cellular response to L-cysteine [GO:0036346] (biological process) Relationships: is_a cellular response to amino acid stimulus [GO:0071230]; is a type of response to L-cysteine [GO:1901367]; is a type of cellular response to nitrogen compound [GO:1901699]; is a type of cellular response to oxygen-containing compound [GO:1901701] Sources: GOC:al Definition: Any process that results in a change in state or activity of a cell (in terms of movement, secretion, enzyme production, gene expression, etc.) as a result of a L-cysteine stimulus. L-cysteine is an optically active form of cysteine having L-configuration.